{
  "term_id": "UNKNOWN:0001",
  "gene_name": "Cytochrome P450 20A1",
  "gene": "UniProtKB:Q6UW02",
  "gene_symbol": "CYP20A1",
  "term_label": "Unknown molecular function"
}